{
  "gene": "UniProtKB:Q96A05",
  "gene_name": "V-type proton ATPase subunit E 2",
  "term_id": "UNKNOWN:0003",
  "term_label": "Unknown cellular component",
  "gene_symbol": "ATP6V1E2"
}